NOXA-BCL-xl complex [GO:0097146] (cellular component) Relationships: is a type of Bcl-2 family protein complex [GO:0097136] References: PMID:14634621 Sources: GOC:so Definition: A heterodimeric protein complex consisting of NOXA and BCL-xl, members of the Bcl-2 family of anti- and proapoptotic regulators.